{
  "term_label": "nucleus",
  "gene_symbol": "DUX4L6",
  "term_id": "GO:0005634",
  "gene_name": "Double homeobox protein 4-like protein 6",
  "gene": "UniProtKB:P0CJ89"
}